{
  "term_id": "GO:0043171",
  "gene_symbol": "IDE",
  "gene_name": "Insulin-degrading enzyme",
  "gene": "UniProtKB:P14735",
  "term_label": "peptide catabolic process"
}